{
  "gene_symbol": "NAP1L2",
  "term_label": "nucleosome assembly",
  "gene_name": "Nucleosome assembly protein 1-like 2",
  "gene": "UniProtKB:Q9ULW6",
  "term_id": "GO:0006334"
}